{
  "term_label": "embryonic skeletal system morphogenesis",
  "gene_name": "Homeobox protein Hox-B3",
  "term_id": "GO:0048704",
  "gene": "UniProtKB:P14651",
  "gene_symbol": "HOXB3"
}